{
  "gene": "UniProtKB:A0A1B0GVT2",
  "term_label": "Unknown cellular component",
  "gene_name": "Small integral membrane protein 36",
  "gene_symbol": "SMIM36",
  "term_id": "UNKNOWN:0003"
}